{
  "gene_symbol": "MINK1",
  "gene_name": "Misshapen-like kinase 1",
  "gene": "UniProtKB:Q8N4C8",
  "term_label": "actin cytoskeleton organization",
  "term_id": "GO:0030036"
}